kinase activator activity [GO:0019209] (molecular function) Definition: Binds to and increases the activity of a kinase, an enzyme which catalyzes of the transfer of a phosphate group, usually from ATP, to a substrate molecule. Subtypes: GO:0030295, GO:0098744 Relationships: is a type of enzyme activator activity [GO:0008047]; is a type of kinase regulator activity [GO:0019207]; positively regulates GO:0016301 Sources: GOC:ai